{
  "gene_symbol": "GLTPD2",
  "gene_name": "Glycolipid transfer protein domain-containing protein 2",
  "term_label": "cytosol",
  "gene": "UniProtKB:A6NH11",
  "term_id": "GO:0005829"
}